metalloexopeptidase activity [GO:0008235] (molecular function) Sources: GOC:mah, https://www.ebi.ac.uk/merops/about/glossary.shtml Subtypes: GO:0004181, metalloaminopeptidase activity [GO:0070006], metallodipeptidase activity [GO:0070573] Relationships: is a type of metallopeptidase activity [GO:0008237]; is a type of GO:0008238 Definition: Catalysis of the hydrolysis of a peptide bond not more than three residues from the N- or C-terminus of a polypeptide chain by a mechanism in which water acts as a nucleophile, one or two metal ions hold the water molecule in place, and charged amino acid side chains are ligands for the metal ions.